maintenance of epithelial integrity, open tracheal system [GO:0035160] (BP) References: PMID:10694415, PMID:14681183 Sources: GOC:mtg_sensu Also known as: maintenance of tracheal epithelial integrity Definition: Ensuring that tracheal tubes in an open tracheal system maintain their epithelial structure during the cell shape changes and movements that occur during the branching process. Relationships: is a type of epithelial structure maintenance [GO:0010669]; is a type of regulation of tube architecture, open tracheal system [GO:0035152]